response to folic acid [GO:0051593] (biological process) Relationships: is a type of response to vitamin [GO:0033273]; is_a response to nitrogen compound [GO:1901698]; is a type of response to oxygen-containing compound [GO:1901700] Sources: GOC:ai Definition: Any process that results in a change in state or activity of a cell or an organism (in terms of movement, secretion, enzyme production, gene expression, etc.) as a result of a folic acid stimulus. Subtypes: GO:0031318, chemotaxis to folate [GO:0043326], cellular response to folic acid [GO:0071231] Also known as: cellular response to folate, cellular response to vitamin B9